phosphoribosyl 1,2-cyclic phosphate phosphodiesterase activity [GO:0103043] (molecular function) Also known as: 5-phospho-alpha-D-ribosyl 1,2-cyclic phosphate phosphodiesterase activity Sources: EC:3.1.4.55 Definition: Catalysis of the reaction: alpha-D-ribose 1,2-cyclic phosphate 5-phosphate + H2O = alpha-D-ribose 1,5-bisphosphate + H+. Relationships: is a type of GO:0008081